box C/D methylation guide RNP complex [GO:0170050] (cellular component) Relationships: is a type of box C/D RNP complex [GO:0170049] References: PMID:28505386, PMID:30254138 Definition: A ribonucleoprotein complex containing a box C/D type snoRNA and three (Archaea) or four (Eukaryotes) core proteins that is capable of methylation of target RNAs.